{
  "gene_name": "NACHT, LRR and PYD domains-containing protein 1",
  "gene_symbol": "NLRP1",
  "term_label": "intrinsic apoptotic signaling pathway",
  "gene": "UniProtKB:Q9C000",
  "term_id": "GO:0097193"
}